{
  "gene_name": "C-Jun-amino-terminal kinase-interacting protein 4",
  "gene": "UniProtKB:O60271",
  "gene_symbol": "SPAG9",
  "term_id": "GO:0019894",
  "term_label": "kinesin binding"
}